{
  "gene_symbol": "SPATA31A6",
  "term_label": "Unknown biological process",
  "term_id": "UNKNOWN:0002",
  "gene_name": "Spermatogenesis-associated protein 31A6",
  "gene": "UniProtKB:Q5VVP1"
}